{
  "term_label": "cytosol",
  "term_id": "GO:0005829",
  "gene": "UniProtKB:P11766",
  "gene_name": "Alcohol dehydrogenase class-3",
  "gene_symbol": "ADH5"
}